{
  "term_label": "carbohydrate metabolic process",
  "gene_symbol": "B3GAT3",
  "gene_name": "Galactosylgalactosylxylosylprotein 3-beta-glucuronosyltransferase 3",
  "term_id": "GO:0005975",
  "gene": "UniProtKB:O94766"
}